{
  "term_id": "UNKNOWN:0001",
  "term_label": "Unknown molecular function",
  "gene_name": "Nuclear pore complex-interacting protein family member A5",
  "gene_symbol": "NPIPA5",
  "gene": "UniProtKB:E9PKD4"
}